{
  "gene_symbol": "GAK",
  "term_id": "GO:0031982",
  "gene": "UniProtKB:O14976",
  "gene_name": "Cyclin-G-associated kinase",
  "term_label": "vesicle"
}